regulation of DNA-templated transcription [GO:0006355] (biological process) Subtypes: GO:0000409, GO:0006356, regulation of transcription by RNA polymerase II [GO:0006357], regulation of transcription by RNA polymerase III [GO:0006359], regulation of mating-type specific transcription, DNA-templated [GO:0007532], regulation of DNA-templated transcription elongation [GO:0032784], negative regulation of DNA-templated transcription [GO:0045892], positive regulation of DNA-templated transcription [GO:0045893], carbon catabolite regulation of transcription [GO:0045990], regulation of transcription by glucose [GO:0046015], regulation of DNA-binding transcription factor activity [GO:0051090], regulation of antisense RNA transcription [GO:0060194], GO:0090293, GO:0140542, regulation of lncRNA transcription [GO:0140743], regulation of miRNA transcription [GO:1902893], regulation of mitochondrial transcription [GO:1903108], regulation of transcription by RNA polymerase V [GO:1904279], regulation of DNA-templated transcription initiation [GO:2000142] Sources: GOC:go_curators, GOC:txnOH Relationships: is a type of GO:0010468; is a type of regulation of RNA biosynthetic process [GO:2001141]; regulates DNA-templated transcription [GO:0006351] Definition: Any process that modulates the frequency, rate or extent of cellular DNA-templated transcription. Also known as: transcriptional control, regulation of cellular transcription, DNA-dependent, regulation of transcription, DNA-dependent, regulation of transcription, DNA-templated, regulation of gene-specific transcription